{
  "term_label": "Unknown cellular component",
  "term_id": "UNKNOWN:0003",
  "gene": "UniProtKB:A0A8V8TLY5",
  "gene_symbol": "A0A8V8TLY5",
  "gene_name": "Ig-like domain-containing protein (Fragment)"
}